{
  "gene_symbol": "PHF1",
  "term_label": "chromatin binding",
  "gene": "UniProtKB:O43189",
  "gene_name": "PHD finger protein 1",
  "term_id": "GO:0003682"
}